{
  "gene": "UniProtKB:Q9BRT3",
  "term_id": "UNKNOWN:0001",
  "gene_name": "Migration and invasion enhancer 1",
  "gene_symbol": "MIEN1",
  "term_label": "Unknown molecular function"
}